{
  "term_label": "Unknown molecular function",
  "term_id": "UNKNOWN:0001",
  "gene_name": "Fas apoptotic inhibitory molecule 1",
  "gene": "UniProtKB:Q9NVQ4",
  "gene_symbol": "FAIM"
}